{
  "gene_symbol": "SPOUT1",
  "gene_name": "Putative methyltransferase C9orf114",
  "gene": "UniProtKB:Q5T280",
  "term_id": "GO:0035198",
  "term_label": "miRNA binding"
}